positive regulation of ribonucleoprotein complex localization [GO:2000199] (biological process) Relationships: is a type of positive regulation of cellular process [GO:0048522]; is a type of GO:2000197; positively regulates ribonucleoprotein complex localization [GO:0071166] Sources: GOC:mah Subtypes: positive regulation of ribosomal subunit export from nucleus [GO:2000202], GO:2000240 Also known as: positive regulation of RNP localization, positive regulation of cellular ribonucleoprotein complex localization, positive regulation of establishment and maintenance of ribonucleoprotein complex localization, positive regulation of ribonucleoprotein complex localisation Definition: Any process that activates or increases the frequency, rate or extent of ribonucleoprotein complex localization.